U1 snRNP binding [GO:1990446] (molecular function) Relationships: is a type of snRNP binding [GO:0070990] References: PMID:14713954 Definition: Binding to a U1 small nuclear ribonucleoprotein particle.